{
  "term_label": "canonical Wnt signaling pathway",
  "gene_symbol": "DVL1",
  "gene": "UniProtKB:O14640",
  "term_id": "GO:0060070",
  "gene_name": "Segment polarity protein dishevelled homolog DVL-1"
}